{
  "gene_name": "7-dehydrocholesterol reductase",
  "gene": "UniProtKB:Q9UBM7",
  "term_label": "cholesterol biosynthetic process",
  "term_id": "GO:0006695",
  "gene_symbol": "DHCR7"
}